cellular response to fluoxetine [GO:0071411] (BP) Definition: Any process that results in a change in state or activity of a cell (in terms of movement, secretion, enzyme production, gene expression, etc.) as a result of a fluoxetine stimulus. Fluoxetine increases the extracellular level of the neurotransmitter serotonin by inhibiting its reuptake into the presynaptic cell, increasing the level of serotonin available to bind to the postsynaptic receptor. Relationships: is a type of GO:0014076; is a type of cellular response to chemical stimulus [GO:0070887] Sources: GOC:mah, GOC:pr Note: Note that this term is in the subset of terms that should not be used for direct manual annotation of gene products. Direct annotations to this term may be amended during annotation QC.